{
  "gene": "UniProtKB:Q96G01",
  "gene_symbol": "BICD1",
  "term_label": "regulation of microtubule cytoskeleton organization",
  "term_id": "GO:0070507",
  "gene_name": "Protein bicaudal D homolog 1"
}